{
  "term_label": "central nervous system development",
  "gene": "UniProtKB:P78509",
  "gene_symbol": "RELN",
  "gene_name": "Reelin",
  "term_id": "GO:0007417"
}